{
  "gene_name": "GTPase ERas",
  "gene": "UniProtKB:Q7Z444",
  "term_label": "plasma membrane",
  "gene_symbol": "ERAS",
  "term_id": "GO:0005886"
}